{
  "gene_symbol": "ARRB2",
  "gene_name": "Beta-arrestin-2",
  "term_id": "GO:0031701",
  "term_label": "angiotensin receptor binding",
  "gene": "UniProtKB:P32121"
}